{
  "gene_name": "RalBP1-associated Eps domain-containing protein 1",
  "gene": "UniProtKB:Q96D71",
  "term_label": "endocytosis",
  "term_id": "GO:0006897",
  "gene_symbol": "REPS1"
}